anchoring junction [GO:0070161] (cellular component) Also known as: anchoring cell junction Subtypes: cell-cell junction [GO:0005911], cell-substrate junction [GO:0030055], flagellum attachment zone [GO:0120119] Definition: A cell junction that mechanically attaches a cell (and its cytoskeleton) to neighboring cells or to the extracellular matrix. Relationships: is a type of GO:0030054 Sources: ISBN:0815332181